{
  "gene": "UniProtKB:Q8IVB4",
  "term_label": "recycling endosome",
  "gene_symbol": "SLC9A9",
  "gene_name": "Sodium_hydrogen exchanger 9",
  "term_id": "GO:0055037"
}